{
  "gene_name": "Zinc finger protein 644",
  "term_label": "regulation of transcription by RNA polymerase II",
  "gene": "UniProtKB:Q9H582",
  "gene_symbol": "ZNF644",
  "term_id": "GO:0006357"
}